{
  "term_label": "plasma membrane",
  "gene": "UniProtKB:Q15334",
  "gene_name": "Lethal(2) giant larvae protein homolog 1",
  "gene_symbol": "LLGL1",
  "term_id": "GO:0005886"
}